interleukin-12 receptor activity [GO:0016517] (molecular function) Definition: Combining with interleukin-12 and transmitting the signal from one side of the membrane to the other to initiate a change in cell activity. Sources: GOC:jl, GOC:signaling Also known as: IL-12 receptor activity, IL-12R Relationships: is a type of GO:0004896; BFO_0000050 GO:0035722; has part interleukin-12 binding [GO:0019972]